{
  "term_label": "nuclear mRNA surveillance of mRNA 3'-end processing",
  "gene_symbol": "ZCCHC7",
  "gene_name": "Zinc finger CCHC domain-containing protein 7",
  "gene": "UniProtKB:Q8N3Z6",
  "term_id": "GO:0071031"
}